triose phosphate transmembrane transport [GO:0035436] (biological process) Note: Note that this term is not intended for use in annotating lateral movement within membranes. Relationships: is a type of GO:0015711; is a type of triose phosphate transport [GO:0015717]; is a type of transmembrane transport [GO:0055085] Also known as: triose phosphate membrane transport Sources: GOC:bf, ISBN:0198506732 Definition: The process in which triose phosphate (glyceraldehyde 3-phosphate) is transported across a membrane. Glyceraldehyde 3-phosphate is any organic three carbon compound phosphate ester.